{
  "term_label": "protein targeting to membrane",
  "gene_name": "Receptor-transporting protein 3",
  "gene": "UniProtKB:Q9BQQ7",
  "gene_symbol": "RTP3",
  "term_id": "GO:0006612"
}